{
  "gene": "UniProtKB:Q08345",
  "gene_name": "Epithelial discoidin domain-containing receptor 1",
  "gene_symbol": "DDR1",
  "term_id": "GO:0005518",
  "term_label": "collagen binding"
}